snRNA catabolic process [GO:0016076] (biological process) Subtypes: nuclear polyadenylation-dependent snRNA catabolic process [GO:0071037] Relationships: is a type of RNA catabolic process [GO:0006401]; is a type of snRNA metabolic process [GO:0016073] Definition: The chemical reactions and pathways resulting in the breakdown of snRNA, small nuclear RNA, low-molecular-mass RNA molecules found in the eukaryotic nucleus as components of the small nuclear ribonucleoprotein. Also known as: snRNA breakdown, snRNA catabolism, snRNA degradation Sources: ISBN:0198506732